{
  "term_id": "GO:0043001",
  "gene_symbol": "VAMP5",
  "gene": "UniProtKB:O95183",
  "term_label": "Golgi to plasma membrane protein transport",
  "gene_name": "Vesicle-associated membrane protein 5"
}